{
  "gene": "UniProtKB:Q96JC9",
  "gene_name": "ELL-associated factor 1",
  "gene_symbol": "EAF1",
  "term_label": "transcription elongation by RNA polymerase II",
  "term_id": "GO:0006368"
}